protein hydroxylation [GO:0018126] (biological process) Sources: GOC:ai Subtypes: peptidyl-lysine hydroxylation [GO:0017185], GO:0018336, peptidyl-proline hydroxylation [GO:0019511], peptidyl-aspartic acid hydroxylation [GO:0042264] Relationships: is a type of GO:0036211 Definition: The addition of a hydroxy group to a protein amino acid. Also known as: protein amino acid hydroxylation